{
  "gene": "UniProtKB:P12319",
  "term_label": "IgE binding",
  "gene_symbol": "FCER1A",
  "term_id": "GO:0019863",
  "gene_name": "High affinity immunoglobulin epsilon receptor subunit alpha"
}